{
  "gene_name": "Progressive ankylosis protein homolog",
  "gene": "UniProtKB:Q9HCJ1",
  "term_id": "GO:0005886",
  "term_label": "plasma membrane",
  "gene_symbol": "ANKH"
}